{
  "gene_name": "Ras-related protein Rab-12",
  "gene": "UniProtKB:Q6IQ22",
  "term_label": "synaptic vesicle",
  "gene_symbol": "RAB12",
  "term_id": "GO:0008021"
}